{
  "term_label": "centrosome",
  "gene_name": "Spindle and centriole-associated protein 1",
  "gene_symbol": "SPICE1",
  "term_id": "GO:0005813",
  "gene": "UniProtKB:Q8N0Z3"
}